chondrocyte morphogenesis involved in endochondral bone morphogenesis [GO:0003414] (BP) Sources: GOC:ascb_2009, GOC:dph, GOC:tb Relationships: is_a GO:0090171; is part of chondrocyte development involved in endochondral bone morphogenesis [GO:0003433] Subtypes: growth plate cartilage chondrocyte morphogenesis [GO:0003429] Definition: The process in which the structures of a chondrocyte that will contribute to bone development are generated and organized.